ATP biosynthetic process [GO:0006754] (biological process) Also known as: ATP anabolism, ATP biosynthesis, ATP formation, ATP synthesis, ATP regeneration Relationships: is a type of purine ribonucleotide biosynthetic process [GO:0009152]; is a type of purine ribonucleoside triphosphate biosynthetic process [GO:0009206]; is a type of GO:0046034 Subtypes: GO:0006756, proton motive force-driven ATP synthesis [GO:0015986] Regulation: regulated by regulation of ATP biosynthetic process [GO:2001169]; negatively regulated by negative regulation of ATP biosynthetic process [GO:2001170]; positively regulated by positive regulation of ATP biosynthetic process [GO:2001171] Definition: The chemical reactions and pathways resulting in the formation of ATP, adenosine 5'-triphosphate, a universally important coenzyme and enzyme regulator. Sources: GOC:go_curators, ISBN:0198506732